{
  "term_id": "GO:0007204",
  "term_label": "positive regulation of cytosolic calcium ion concentration",
  "gene_symbol": "PTGER4",
  "gene": "UniProtKB:P35408",
  "gene_name": "Prostaglandin E2 receptor EP4 subtype"
}